tryptophan transport [GO:0015827] (biological process) Also known as: L-tryptophan transport Sources: GOC:ai Definition: The directed movement of tryptophan, 2-amino-3-(1H-indol-3-yl)propanoic acid, into, out of or within a cell, or between cells, by means of some agent such as a transporter or pore. Relationships: is a type of GO:0006865; is a type of organic cation transport [GO:0015695]; is a type of aromatic amino acid transport [GO:0015801] Subtypes: L-tryptophan transmembrane transport [GO:1904556]